{
  "gene_symbol": "HDAC7",
  "term_id": "GO:0040029",
  "gene_name": "Histone deacetylase 7",
  "gene": "UniProtKB:Q8WUI4",
  "term_label": "epigenetic regulation of gene expression"
}